positive regulation of dopamine metabolic process [GO:0045964] (biological process) Definition: Any process that activates or increases the frequency, rate or extent of the chemical reactions and pathways involving dopamine. Subtypes: positive regulation of dopamine biosynthetic process [GO:1903181] Sources: GOC:go_curators Relationships: is a type of positive regulation of amine metabolic process [GO:0033240]; is a type of regulation of dopamine metabolic process [GO:0042053]; RO_0002213 dopamine metabolic process [GO:0042417] Also known as: positive regulation of dopamine metabolism, up regulation of dopamine metabolic process, up-regulation of dopamine metabolic process, upregulation of dopamine metabolic process, activation of dopamine metabolic process, stimulation of dopamine metabolic process